cell fate determination involved in pattern specification [GO:0060582] (biological process) Subtypes: GO:0016360, ventral spinal cord interneuron fate determination [GO:0060580] Relationships: is a type of cell fate determination [GO:0001709]; is part of GO:0060581 Sources: GOC:dph Definition: A process involved in commitment of a cell to a fate in a developmental field. Once determination has taken place, a cell becomes committed to differentiate down a particular pathway regardless of its environment.